{
  "gene": "UniProtKB:Q9H900",
  "gene_name": "Protein zwilch homolog",
  "term_id": "GO:0007094",
  "term_label": "mitotic spindle assembly checkpoint signaling",
  "gene_symbol": "ZWILCH"
}